{
  "gene": "UniProtKB:P51397",
  "gene_symbol": "DAP",
  "term_label": "ribosome binding",
  "term_id": "GO:0043022",
  "gene_name": "Death-associated protein 1"
}